{
  "gene_symbol": "UBE4A",
  "term_id": "GO:0034450",
  "gene_name": "Ubiquitin conjugation factor E4 A",
  "gene": "UniProtKB:Q14139",
  "term_label": "ubiquitin-ubiquitin ligase activity"
}